{
  "gene": "UniProtKB:Q93099",
  "term_id": "GO:0004411",
  "term_label": "homogentisate 1,2-dioxygenase activity",
  "gene_symbol": "HGD",
  "gene_name": "Homogentisate 1,2-dioxygenase"
}